{
  "gene": "UniProtKB:P29373",
  "gene_symbol": "CRABP2",
  "gene_name": "Cellular retinoic acid-binding protein 2",
  "term_id": "GO:0005504",
  "term_label": "fatty acid binding"
}